{
  "gene_name": "Sodium channel protein type 4 subunit alpha",
  "gene": "UniProtKB:P35499",
  "term_label": "sodium ion transmembrane transport",
  "term_id": "GO:0035725",
  "gene_symbol": "SCN4A"
}